{
  "gene_symbol": "ACTG1",
  "term_label": "structural constituent of postsynaptic actin cytoskeleton",
  "gene": "UniProtKB:P63261",
  "gene_name": "Actin, cytoplasmic 2",
  "term_id": "GO:0098973"
}